{
  "gene_name": "Histone deacetylase 11",
  "term_label": "epigenetic regulation of gene expression",
  "gene": "UniProtKB:Q96DB2",
  "gene_symbol": "HDAC11",
  "term_id": "GO:0040029"
}